{
  "term_label": "Unknown molecular function",
  "gene_symbol": "LYPD3",
  "gene": "UniProtKB:O95274",
  "gene_name": "Ly6_PLAUR domain-containing protein 3",
  "term_id": "UNKNOWN:0001"
}